{
  "gene_symbol": "EFNA1",
  "gene_name": "Ephrin-A1",
  "term_label": "ephrin receptor signaling pathway",
  "term_id": "GO:0048013",
  "gene": "UniProtKB:P20827"
}